{
  "term_label": "F-actin capping protein complex",
  "term_id": "GO:0008290",
  "gene_name": "F-actin-capping protein subunit alpha-1",
  "gene": "UniProtKB:P52907",
  "gene_symbol": "CAPZA1"
}